{
  "term_label": "plasma membrane",
  "term_id": "GO:0005886",
  "gene_name": "Ras-related protein Rap-1A",
  "gene": "UniProtKB:P62834",
  "gene_symbol": "RAP1A"
}